{
  "term_label": "fatty acid binding",
  "gene": "UniProtKB:Q5NUL3",
  "gene_symbol": "FFAR4",
  "gene_name": "Free fatty acid receptor 4",
  "term_id": "GO:0005504"
}